{
  "term_id": "GO:0044528",
  "gene_symbol": "FASTKD1",
  "term_label": "regulation of mitochondrial mRNA stability",
  "gene_name": "FAST kinase domain-containing protein 1, mitochondrial",
  "gene": "UniProtKB:Q53R41"
}